tRNA pseudouridine(55) synthase activity [GO:0160148] (molecular function) Definition: Catalysis of the reaction: uridine(55) in tRNA = pseudouridine(55) in tRNA. Sources: EC:5.4.99.25 Relationships: is a type of tRNA pseudouridine synthase activity [GO:0106029]